{
  "gene_name": "pre-mRNA 3' end processing protein WDR33",
  "term_label": "Unknown biological process",
  "gene_symbol": "WDR33",
  "gene": "UniProtKB:Q9C0J8",
  "term_id": "UNKNOWN:0002"
}